acetyl CoA:(Z)-3-hexen-1-ol acetyltransferase activity [GO:0010327] (molecular function) Relationships: is a type of GO:0016413 Definition: Catalysis of the reaction: acetyl-CoA + (Z)-3-hexen-1-ol = CoA + (Z)-3-hexen-1-yl acetate. Also known as: hexenol acetyltransferase References: PMID:17163883